{
  "term_label": "nuclear pore outer ring",
  "gene_name": "Nuclear pore complex protein Nup107",
  "gene": "UniProtKB:P57740",
  "gene_symbol": "NUP107",
  "term_id": "GO:0031080"
}